{
  "gene_name": "MKRN2 opposite strand protein",
  "term_label": "Unknown cellular component",
  "gene_symbol": "MKRN2OS",
  "gene": "UniProtKB:H3BPM6",
  "term_id": "UNKNOWN:0003"
}